{
  "gene": "UniProtKB:P0DP24",
  "gene_symbol": "CALM2",
  "term_id": "GO:0097720",
  "term_label": "calcineurin-mediated signaling",
  "gene_name": "Calmodulin-2"
}